{
  "term_id": "GO:0005886",
  "gene": "UniProtKB:Q9NPG4",
  "gene_name": "Protocadherin-12",
  "gene_symbol": "PCDH12",
  "term_label": "plasma membrane"
}